regulation of protein ADP-ribosylation [GO:0010835] (biological process) Definition: Any process that modulates the frequency, rate or extent of protein ADP-ribosylation. Protein ADP-ribosylation is the transfer, from NAD, of ADP-ribose to protein amino acids. Sources: GOC:dph, GOC:tb Also known as: regulation of protein amino acid ADP-ribosylation Relationships: is a type of regulation of transferase activity [GO:0051338]; regulates NAD+-protein mono-ADP-ribosyltransferase activity [GO:1990404] Subtypes: GO:0010836